{
  "gene_symbol": "TUBA4B",
  "term_label": "Unknown cellular component",
  "gene": "UniProtKB:Q9H853",
  "term_id": "UNKNOWN:0003",
  "gene_name": "Putative tubulin-like protein alpha-4B"
}